regulation of signal transduction [GO:0009966] (BP) Sources: GOC:sm Subtypes: regulation of cytokine-mediated signaling pathway [GO:0001959], signal complex assembly [GO:0007172], regulation of G protein-coupled receptor signaling pathway [GO:0008277], regulation of smoothened signaling pathway [GO:0008589], regulation of Toll signaling pathway [GO:0008592], GO:0008593, GO:0009787, GO:0009937, GO:0009967, GO:0009968, regulation of signaling receptor activity [GO:0010469], regulation of platelet-derived growth factor receptor signaling pathway [GO:0010640], GO:0010928, adaptation of signaling pathway [GO:0023058], regulation of Wnt signaling pathway [GO:0030111], regulation of vascular endothelial growth factor receptor signaling pathway [GO:0030947], regulation of brain-derived neurotrophic factor receptor signaling pathway [GO:0031548], GO:0031664, regulation of Roundabout signaling pathway [GO:0035386], GO:0038009, GO:0040036, regulation of insulin-like growth factor receptor signaling pathway [GO:0043567], regulation of sevenless signaling pathway [GO:0045501], regulation of insulin receptor signaling pathway [GO:0046626], GO:0050854, regulation of neurotrophin TRK receptor signaling pathway [GO:0051386], GO:0060238, regulation of Fc receptor mediated stimulatory signaling pathway [GO:0060368], regulation of growth hormone receptor signaling pathway [GO:0060398], regulation of pattern recognition receptor signaling pathway [GO:0062207], regulation of cytokinin-activated signaling pathway [GO:0080036], regulation of transmembrane receptor protein serine/threonine kinase signaling pathway [GO:0090092], regulation of red or far-red light signaling pathway [GO:0090227], modulation of excitatory postsynaptic potential [GO:0098815], modulation of inhibitory postsynaptic potential [GO:0098828], regulation of torso signaling pathway [GO:0120175], extracellular regulation of signal transduction [GO:1900115], regulation of glutamate receptor signaling pathway [GO:1900449], regulation of brassinosteroid mediated signaling pathway [GO:1900457], regulation of vascular endothelial growth factor signaling pathway [GO:1900746], regulation of ERBB signaling pathway [GO:1901184], regulation of ephrin receptor signaling pathway [GO:1901187], regulation of Fas signaling pathway [GO:1902044], regulation of sphingolipid mediated signaling pathway [GO:1902068], regulation of hepatocyte growth factor receptor signaling pathway [GO:1902202], regulation of intracellular signal transduction [GO:1902531], regulation of glucose mediated signaling pathway [GO:1902659], GO:1902841, GO:1902847, regulation of receptor signaling pathway via STAT [GO:1904892], regulation of apolipoprotein A-I-mediated signaling pathway [GO:1905094], regulation of postsynapse to nucleus signaling pathway [GO:1905539], signal clustering [GO:1990256], regulation of jasmonic acid mediated signaling pathway [GO:2000022], regulation of salicylic acid mediated signaling pathway [GO:2000031], regulation of CD40 signaling pathway [GO:2000348], regulation of glial cell-derived neurotrophic factor receptor signaling pathway involved in ureteric bud formation [GO:2000733], regulation of integrin-mediated signaling pathway [GO:2001044], regulation of apoptotic signaling pathway [GO:2001233], regulation of semaphorin-plexin signaling pathway [GO:2001260] Relationships: is a type of GO:0010646; is a type of regulation of signaling [GO:0023051]; is a type of regulation of response to stimulus [GO:0048583]; regulates signal transduction [GO:0007165] Also known as: regulation of signaling pathway, regulation of signalling pathway Definition: Any process that modulates the frequency, rate or extent of signal transduction.